{
  "gene": "UniProtKB:O43837",
  "term_id": "GO:0006099",
  "gene_symbol": "IDH3B",
  "gene_name": "Isocitrate dehydrogenase [NAD] subunit beta, mitochondrial",
  "term_label": "tricarboxylic acid cycle"
}